regulation of artery smooth muscle contraction [GO:1905654] (BP) Definition: Any process that modulates the frequency, rate or extent of artery smooth muscle contraction. Subtypes: negative regulation of artery smooth muscle contraction [GO:1905655], positive regulation of artery smooth muscle contraction [GO:1905656] References: PMID:27389411 Sources: GOC:BHF, GOC:BHF_miRNA, GOC:TermGenie, GOC:rph, GO_REF:0000058 Relationships: is a type of regulation of vascular associated smooth muscle contraction [GO:0003056]; regulates artery smooth muscle contraction [GO:0014824]